{
  "gene_name": "Spermatogenesis- and oogenesis-specific basic helix-loop-helix-containing protein 2",
  "term_label": "nucleus",
  "gene": "UniProtKB:Q9NX45",
  "gene_symbol": "SOHLH2",
  "term_id": "GO:0005634"
}